{
  "gene_symbol": "SLAMF8",
  "gene_name": "SLAM family member 8",
  "gene": "UniProtKB:Q9P0V8",
  "term_label": "Unknown cellular component",
  "term_id": "UNKNOWN:0003"
}